{
  "term_label": "regulation of transcription by RNA polymerase II",
  "gene": "UniProtKB:Q99853",
  "gene_name": "Forkhead box protein B1",
  "gene_symbol": "FOXB1",
  "term_id": "GO:0006357"
}